photoreactive repair [GO:0000719] (biological process) Definition: The repair of UV-induced T-T, C-T and C-C dimers by directly reversing the damage to restore the original pyrimidines. Also known as: pyrimidine-dimer repair by photolyase References: PMID:10915863 Sources: GOC:elh Relationships: is a type of pyrimidine dimer repair [GO:0006290]